sodium:malonate symporter activity [GO:0044668] (molecular function) Sources: GOC:crds Definition: Enables the transfer of a solute or solutes from one side of a membrane to the other according to the reaction: sodium(out)+ malonate(out) = sodium(in) + malonate(in). Relationships: is a type of sodium:dicarboxylate symporter activity [GO:0017153]; is a type of GO:1901239